mismatched DNA binding [GO:0030983] (molecular function) Relationships: is a type of double-stranded DNA binding [GO:0003690] Subtypes: DNA insertion or deletion binding [GO:0032135], adenine/cytosine mispair binding [GO:0032136], GO:0032137, adenine/adenine mispair binding [GO:0035484], adenine/guanine mispair binding [GO:0035485], GO:0035486, GO:0035487, cytosine/thymine mispair binding [GO:0035488], guanine/guanine mispair binding [GO:0035489] Also known as: mispair binding, mispaired DNA binding Sources: GOC:mah Definition: Binding to a double-stranded DNA region containing one or more mismatches.